glutamic-type peptidase activity [GO:0070002] (molecular function) Subtypes: GO:0070007 Definition: Catalysis of the hydrolysis of peptide bonds in a polypeptide chain by a mechanism involving a glutamate/glutamine catalytic dyad. Relationships: is a type of peptidase activity [GO:0008233] Sources: GOC:mah, https://www.ebi.ac.uk/merops/about/glossary.shtml#CATTYPE